{
  "gene": "UniProtKB:Q9P2G3",
  "term_id": "GO:0043025",
  "gene_symbol": "KLHL14",
  "gene_name": "Kelch-like protein 14",
  "term_label": "neuronal cell body"
}